mucilage biosynthetic process [GO:0010192] (BP) Sources: GOC:sm Also known as: mucilage anabolism, mucilage biosynthesis, mucilage formation, mucilage synthesis Subtypes: GO:0048354, GO:0048355, root epithelial mucilage biosynthetic process [GO:0048356], pedicel mucilage biosynthetic process [GO:0048357] Definition: The chemical reactions and pathways resulting in the formation of mucilage, a gelatinous substance secreted by plants. Relationships: is a type of biosynthetic process [GO:0009058]